{
  "gene": "UniProtKB:Q96N66",
  "term_label": "membrane",
  "gene_name": "Lysophospholipid acyltransferase 7",
  "gene_symbol": "MBOAT7",
  "term_id": "GO:0016020"
}